symbiont-mediated suppression of host complement activation by complement sequestering [GO:0141116] (biological process) Also known as: suppression of complement activation by another organism by complement sequestering Definition: A process by which a symbiont prevents host complement activation by sequestering it away from its surface. References: PMID:18323455 Relationships: is a type of symbiont-mediated suppression of host complement activation [GO:0042784]